{
  "gene_symbol": "MTRNR2L4",
  "gene": "UniProtKB:P0CJ71",
  "term_id": "UNKNOWN:0003",
  "gene_name": "Humanin-like 4",
  "term_label": "Unknown cellular component"
}